{
  "gene_name": "Acetylcholinesterase",
  "gene": "UniProtKB:P22303",
  "term_label": "acetylcholine catabolic process",
  "gene_symbol": "ACHE",
  "term_id": "GO:0006581"
}